{
  "gene_name": "RING1 and YY1-binding protein",
  "term_label": "nucleus",
  "term_id": "GO:0005634",
  "gene": "UniProtKB:Q8N488",
  "gene_symbol": "RYBP"
}